{
  "term_id": "GO:0030424",
  "gene_symbol": "NPTN",
  "gene_name": "Neuroplastin",
  "term_label": "axon",
  "gene": "UniProtKB:Q9Y639"
}